{
  "gene": "UniProtKB:Q6DN90",
  "term_label": "regulation of postsynaptic neurotransmitter receptor internalization",
  "gene_name": "IQ motif and SEC7 domain-containing protein 1",
  "term_id": "GO:0099149",
  "gene_symbol": "IQSEC1"
}